{
  "gene_symbol": "AKAP10",
  "term_label": "mitochondrion",
  "gene": "UniProtKB:O43572",
  "term_id": "GO:0005739",
  "gene_name": "A-kinase anchor protein 10, mitochondrial"
}